myxospore formation [GO:0034303] (biological process) Relationships: is a type of asexual sporulation resulting in formation of a cellular spore [GO:0043936] Sources: GOC:ds, ISBN:0122268008 Definition: The process in which differentiated, resting cells are formed, usually within a fruiting body by Myxobacteria. The myxospore is more resistant to high temperature, desiccation, and UV than vegetative myxobacteria.